{
  "gene": "UniProtKB:P0DV76",
  "term_label": "Unknown molecular function",
  "term_id": "UNKNOWN:0001",
  "gene_symbol": "FAM90A19",
  "gene_name": "Protein FAM90A19"
}